{
  "gene": "UniProtKB:Q86YR6",
  "term_id": "UNKNOWN:0003",
  "gene_name": "POTE ankyrin domain family member D",
  "gene_symbol": "POTED",
  "term_label": "Unknown cellular component"
}